{
  "gene_symbol": "SUOX",
  "gene": "UniProtKB:P51687",
  "term_label": "sulfite oxidase activity",
  "gene_name": "Sulfite oxidase, mitochondrial",
  "term_id": "GO:0008482"
}